sphingolipid translocation [GO:0099039] (biological process) Relationships: is a type of lipid translocation [GO:0034204]; is_a nitrogen compound transport [GO:0071705] Subtypes: ceramide translocation [GO:0099040] Sources: GOC:BHF, GOC:rl Definition: The movement of a sphingolipid molecule from one leaflet of a membrane bilayer to the opposite leaflet.